{
  "gene_name": "Secreted Ly-6_uPAR-related protein 1",
  "term_label": "Unknown biological process",
  "gene": "UniProtKB:P55000",
  "gene_symbol": "SLURP1",
  "term_id": "UNKNOWN:0002"
}